{
  "term_id": "GO:0005739",
  "gene": "UniProtKB:Q9H1A3",
  "term_label": "mitochondrion",
  "gene_name": "Protein-L-histidine N-pros-methyltransferase",
  "gene_symbol": "METTL9"
}